host cell rough endoplasmic reticulum [GO:0044168] (cellular component) Definition: The irregular network of unit membranes, visible only by electron microscopy, that occurs in the host cell cytoplasm of many eukaryotic cells. The membranes form a complex meshwork of tubular channels, which are often expanded into slitlike cavities called cisternae. The host rough ER has ribosomes adhering to the outer surface. Also known as: host rough endoplasmic reticulum Sources: GOC:jl Relationships: is a type of GO:0044165